DPS complex [GO:1990567] (cellular component) Definition: A protein serine/threonine phosphatase complex that in S. pombe consists of the proteins Dis2, Ppn1, and Swd22. Relationships: is a type of protein serine/threonine phosphatase complex [GO:0008287] References: PMID:24945319